melanin-concentrating hormone activity [GO:0030354] (molecular function) References: PMID:11416225, PMID:9792536 Sources: GOC:mah Relationships: is a type of hormone activity [GO:0005179] Definition: The action characteristic of melanin-concentrating hormone, a cyclic peptide hormone that, upon receptor binding, induces melanin aggregation in melanocytes, and is also involved in regulating food intake and energy balance in mammals.